{
  "gene": "UniProtKB:Q9NZI2",
  "term_id": "GO:1901379",
  "gene_symbol": "KCNIP1",
  "term_label": "regulation of potassium ion transmembrane transport",
  "gene_name": "Kv channel-interacting protein 1"
}